MutLbeta complex binding [GO:0032406] (molecular function) Sources: GOC:vk Relationships: is a type of mismatch repair complex binding [GO:0032404] Definition: Binding to a MutLbeta mismatch repair complex.